{
  "term_label": "Unknown cellular component",
  "gene": "UniProtKB:Q9NRJ1",
  "gene_name": "Protein MOST-1",
  "gene_symbol": "C8orf17",
  "term_id": "UNKNOWN:0003"
}